cell cycle switching [GO:0060184] (biological process) Subtypes: GO:0051728 Sources: GOC:dph, GOC:kmv, GOC:tb Definition: The process in which a cell switches cell cycle mode. Relationships: is a type of cell cycle process [GO:0022402]